intraciliary transport particle A [GO:0030991] (cellular component) Relationships: is a type of protein-containing complex [GO:0032991]; is part of GO:0030990 Also known as: intraflagellar transport complex A, intraflagellar transport particle A, IFT A complex, IFT complex A Definition: The smaller subcomplex of the intraciliary transport particle; characterized complexes have molecular weights of 710-760 kDa. Note: Note that we deem cilia and microtubule-based flagella to be equivalent. References: PMID:14570576 Sources: GOC:cilia, GOC:kmv